{
  "gene_symbol": "RPL29",
  "gene_name": "Large ribosomal subunit protein eL29",
  "term_label": "structural constituent of ribosome",
  "term_id": "GO:0003735",
  "gene": "UniProtKB:P47914"
}